{
  "gene_symbol": "WNK4",
  "term_label": "signal transduction",
  "gene_name": "Serine_threonine-protein kinase WNK4",
  "gene": "UniProtKB:Q96J92",
  "term_id": "GO:0007165"
}